mannosyl-oligosaccharide 1,2-alpha-mannosidase activity [GO:0004571] (molecular function) Definition: Catalysis of the hydrolysis of the terminal (1->2)-linked alpha-D-mannose residues in an oligo-mannose oligosaccharide. Also known as: Man9-mannosidase activity, ManI activity, mannose-9 processing alpha-mannosidase activity, mannosidase 1A activity, mannosidase 1B activity, 1,2-alpha-mannosidase, 1,2-alpha-mannosyl-oligosaccharide alpha-D-mannohydrolase activity, exo-alpha-1,2-mannanase activity, glycoprotein processing mannosidase I, mannosidase I References: PMID:25092655 Sources: GOC:bf Relationships: is a type of mannosyl-oligosaccharide mannosidase activity [GO:0015924]